N-acetyl-beta-alanine deacetylase activity [GO:0050117] (molecular function) Definition: Catalysis of the reaction: N-acetyl-beta-alanine + H2O = beta-alanine + acetate. Sources: EC:3.5.1.21, RHEA:23212 Also known as: N-acetyl-beta-alanine amidohydrolase activity Relationships: is a type of hydrolase activity, acting on carbon-nitrogen (but not peptide) bonds, in linear amides [GO:0016811]; is a type of deacetylase activity [GO:0019213]